positive regulation of dendritic cell cytokine production [GO:0002732] (biological process) Sources: GOC:add Also known as: up regulation of dendritic cell cytokine production, up-regulation of dendritic cell cytokine production, upregulation of dendritic cell cytokine production, activation of dendritic cell cytokine production, stimulation of dendritic cell cytokine production Subtypes: positive regulation of myeloid dendritic cell cytokine production [GO:0002735], positive regulation of plasmacytoid dendritic cell cytokine production [GO:0002738] Definition: Any process that activates or increases the frequency, rate, or extent of dendritic cell cytokine production. Relationships: is a type of GO:0002705; is a type of positive regulation of cytokine production involved in immune response [GO:0002720]; is a type of regulation of dendritic cell cytokine production [GO:0002730]; positively regulates dendritic cell cytokine production [GO:0002371]